{
  "term_id": "GO:0005667",
  "gene": "UniProtKB:Q9ULK4",
  "gene_name": "Mediator of RNA polymerase II transcription subunit 23",
  "gene_symbol": "MED23",
  "term_label": "transcription regulator complex"
}